{
  "term_label": "hormone-mediated signaling pathway",
  "gene_name": "Growth hormone secretagogue receptor type 1",
  "gene": "UniProtKB:Q92847",
  "gene_symbol": "GHSR",
  "term_id": "GO:0009755"
}